{
  "term_id": "GO:0031012",
  "gene": "UniProtKB:O15232",
  "term_label": "extracellular matrix",
  "gene_symbol": "MATN3",
  "gene_name": "Matrilin-3"
}